{
  "gene_symbol": "C1orf167",
  "gene_name": "Uncharacterized protein C1orf167",
  "term_id": "UNKNOWN:0001",
  "term_label": "Unknown molecular function",
  "gene": "UniProtKB:Q5SNV9"
}